{
  "term_label": "Unknown cellular component",
  "gene_name": "Thyroid adenoma-associated protein",
  "gene_symbol": "THADA",
  "term_id": "UNKNOWN:0003",
  "gene": "UniProtKB:Q6YHU6"
}